spontaneous synaptic transmission [GO:0098814] (BP) Note: This is typically measured via detection of mini excitatory post-synaptic currents (mEPSCs). Definition: The low level of synaptic transmission that occurs via spontaneous neurotransmitter release into the synaptic cleft in the absence of a presynaptic action potential. Also known as: basal synaptic transmission Relationships: is a type of chemical synaptic transmission [GO:0007268]; has part spontaneous neurotransmitter secretion [GO:0061669] Regulation: regulated by GO:0150003 References: PMID:20200227